{
  "term_id": "GO:0002181",
  "term_label": "cytoplasmic translation",
  "gene_symbol": "RPL36",
  "gene": "UniProtKB:Q9Y3U8",
  "gene_name": "Large ribosomal subunit protein eL36"
}